dorsal closure, leading edge cell fate commitment [GO:0035029] (biological process) Relationships: is a type of GO:0035027; is part of GO:0046663 Sources: GOC:bf Definition: The commitment of cells to leading edge cell fate during dorsal closure. Leading edge cells are the dorsal-most cells of the migrating epidermis.